{
  "term_id": "GO:0031573",
  "gene": "UniProtKB:Q6WBX8",
  "gene_name": "Cell cycle checkpoint control protein RAD9B",
  "term_label": "mitotic intra-S DNA damage checkpoint signaling",
  "gene_symbol": "RAD9B"
}